modified amino acid catabolic process [GO:0042219] (biological process) Also known as: amino acid derivative catabolic process, cellular amino acid derivative breakdown, cellular amino acid derivative catabolic process, cellular amino acid derivative catabolism, cellular amino acid derivative degradation, cellular modified amino acid breakdown, cellular modified amino acid catabolic process, cellular modified amino acid catabolism, cellular modified amino acid degradation, modified amino acid catabolism Subtypes: amino-acid betaine catabolic process [GO:0006579], phosphatidylserine catabolic process [GO:0006660], GO:0006751, GO:0009397, pantothenate catabolic process [GO:0015941], trans-4-hydroxy-L-proline catabolic process [GO:0019470], S-adenosylhomocysteine catabolic process [GO:0019510], GO:0030328, phosphagen catabolic process [GO:0042397], thyroid hormone catabolic process [GO:0042404], hydroxylysine catabolic process [GO:0046948], modified histidine catabolic process [GO:0052702], ochratoxin A catabolic process [GO:1900817], sarcosine catabolic process [GO:1901053], lincomycin catabolic process [GO:1901773], N(omega)-methyl-L-arginine catabolic process [GO:2001297], N(omega),N(omega)-dimethyl-L-arginine catabolic process [GO:2001299] Relationships: is a type of modified amino acid metabolic process [GO:0006575]; is a type of catabolic process [GO:0009056] Sources: GOC:ai Definition: The chemical reactions and pathways resulting in the breakdown of compounds derived from amino acids, organic acids containing one or more amino substituents.